{
  "gene_name": "Volume-regulated anion channel subunit LRRC8D",
  "gene": "UniProtKB:Q7L1W4",
  "gene_symbol": "LRRC8D",
  "term_id": "GO:0015810",
  "term_label": "aspartate transmembrane transport"
}